{
  "gene": "UniProtKB:Q6ZUT6",
  "term_id": "UNKNOWN:0002",
  "term_label": "Unknown biological process",
  "gene_name": "Coiled-coil domain-containing protein 9B",
  "gene_symbol": "CCDC9B"
}